{
  "gene_symbol": "TMEM241",
  "gene": "UniProtKB:Q24JQ0",
  "term_label": "Golgi apparatus",
  "term_id": "GO:0005794",
  "gene_name": "Transmembrane protein 241"
}